{
  "term_id": "UNKNOWN:0002",
  "gene": "UniProtKB:Q8N660",
  "term_label": "Unknown biological process",
  "gene_symbol": "NBPF15",
  "gene_name": "Neuroblastoma breakpoint family member 15"
}